ligase activity, forming phosphoric ester bonds [GO:0016886] (molecular function) Sources: EC:6.5.-.- Definition: Catalysis of the joining of two molecules, or two groups within a single molecule, via a phosphoric ester bond, with the concomitant hydrolysis of the diphosphate bond in ATP or a similar triphosphate. Subtypes: DNA ligase activity [GO:0003909], RNA-3'-phosphate cyclase activity [GO:0003963], RNA ligase activity [GO:0008452], peptide lactyltransferase (ATP-dependent) activity [GO:0141207] Relationships: is_a GO:0016874